{
  "term_id": "GO:1902808",
  "gene_symbol": "FAM83D",
  "gene_name": "Protein FAM83D",
  "gene": "UniProtKB:Q9H4H8",
  "term_label": "positive regulation of cell cycle G1/S phase transition"
}